{
  "gene_symbol": "JAK2",
  "term_id": "GO:0042981",
  "gene_name": "Tyrosine-protein kinase JAK2",
  "term_label": "regulation of apoptotic process",
  "gene": "UniProtKB:O60674"
}